regulation of DNA damage response, signal transduction by p53 class mediator [GO:0043516] (biological process) Sources: GOC:jl Relationships: is a type of regulation of cellular response to stress [GO:0080135]; is a type of regulation of signal transduction by p53 class mediator [GO:1901796]; regulates DNA damage response, signal transduction by p53 class mediator [GO:0030330] Subtypes: GO:0043517, GO:0043518 Also known as: regulation of p53 induced by DNA damage response Definition: Any process that modulates the frequency, rate or extent of the cascade of processes induced by the cell cycle regulator phosphoprotein p53, or an equivalent protein, in response to the detection of DNA damage.